NAD transmembrane transport [GO:0035352] (biological process) Relationships: is a type of NAD transport [GO:0043132]; is a type of purine-containing compound transmembrane transport [GO:0072530]; is a type of nucleotide transmembrane transport [GO:1901679] Definition: The process in which a nicotinamide adenine dinucleotide is transported across a membrane; transport may be of either the oxidized form, NAD, or the reduced form, NADH. Sources: GOC:bf Also known as: NAD membrane transport Subtypes: mitochondrial NAD transmembrane transport [GO:1990549] Note: Note that this term is not intended for use in annotating lateral movement within membranes.